positive regulation of protein localization to chromosome, telomeric region [GO:1904816] (biological process) References: PMID:19487455 Sources: GOC:BHF, GOC:BHF_telomere, GOC:TermGenie, GOC:nc, GO_REF:0000058 Also known as: positive regulation of protein localisation to chromosome, telomeric region, positive regulation of protein localization to telomere, up regulation of protein localisation to chromosome, telomeric region, up regulation of protein localization to chromosome, telomeric region, up regulation of protein localization to telomere, up-regulation of protein localisation to chromosome, telomeric region, up-regulation of protein localization to chromosome, telomeric region, up-regulation of protein localization to telomere, upregulation of protein localisation to chromosome, telomeric region, upregulation of protein localization to chromosome, telomeric region, upregulation of protein localization to telomere, activation of protein localisation to chromosome, telomeric region, activation of protein localization to chromosome, telomeric region, activation of protein localization to telomere Definition: Any process that activates or increases the frequency, rate or extent of protein localization to chromosome, telomeric region. Relationships: is a type of positive regulation of protein localization [GO:1903829]; is_a GO:1904814; positively regulates protein localization to chromosome, telomeric region [GO:0070198]